{
  "gene_symbol": "KLHL41",
  "term_id": "GO:1990756",
  "gene_name": "Kelch-like protein 41",
  "gene": "UniProtKB:O60662",
  "term_label": "ubiquitin-like ligase-substrate adaptor activity"
}